{
  "gene_symbol": "MT-ND3",
  "gene_name": "NADH-ubiquinone oxidoreductase chain 3",
  "term_label": "NADH dehydrogenase (ubiquinone) activity",
  "gene": "UniProtKB:P03897",
  "term_id": "GO:0008137"
}